{
  "term_id": "GO:0008020",
  "gene": "UniProtKB:P04001",
  "gene_name": "Medium-wave-sensitive opsin 1",
  "gene_symbol": "OPN1MW",
  "term_label": "G protein-coupled photoreceptor activity"
}